arachidonate 11,12-epoxygenase activity [GO:0008405] (molecular function) Relationships: is_a arachidonate epoxygenase activity [GO:0008392] Also known as: arachidonic acid 11,12-epoxygenase activity, cytochrome P450 CYP2C38 References: PMID:10681399 Sources: RHEA:51480, http://lipidlibrary.aocs.org/Lipids/eic_hete/index.htm Definition: Catalysis of an NADPH- and oxygen-dependent reaction that converts arachidonic acid to cis-11,12-epoxyeicosatrienoic acid.